{
  "term_label": "nucleus",
  "gene_symbol": "NKX3-2",
  "gene": "UniProtKB:P78367",
  "gene_name": "Homeobox protein Nkx-3.2",
  "term_id": "GO:0005634"
}